ABC-type zinc transporter activity [GO:0015633] (molecular function) Also known as: ATP-dependent zinc transmembrane transporter activity, ATPase-coupled zinc transmembrane transporter activity, zinc transporting ATPase activity, zinc-transporting ATPase activity, zinc porter activity Relationships: is a type of zinc ion transmembrane transporter activity [GO:0005385]; is a type of ATPase-coupled monoatomic cation transmembrane transporter activity [GO:0019829]; is a type of ABC-type transporter activity [GO:0140359] Definition: Enables the transfer of a solute or solutes from one side of a membrane to the other according to the reaction: ATP + H2O + Zn2+(out) = ADP + phosphate + Zn2+(in). Sources: RHEA:29795